vasoconstriction of artery involved in ischemic response to lowering of systemic arterial blood pressure [GO:0002014] (biological process) Definition: The vasoconstriction that is triggered by vasomotor excitation resulting from the detection of high carbon dioxide levels in the vasomotor center of the central nervous system. Sources: GOC:mtg_cardio, ISBN:0721643949 Relationships: is a type of positive regulation of systemic arterial blood pressure [GO:0003084]; is a type of GO:0042310; is part of regulation of systemic arterial blood pressure by ischemic conditions [GO:0001980]